{
  "term_id": "GO:0060326",
  "gene_name": "Atypical chemokine receptor 2",
  "gene_symbol": "ACKR2",
  "term_label": "cell chemotaxis",
  "gene": "UniProtKB:O00590"
}